{
  "term_id": "GO:0000981",
  "gene_name": "Double homeobox protein 4-like protein 2",
  "gene": "UniProtKB:P0CJ85",
  "gene_symbol": "DUX4L2",
  "term_label": "DNA-binding transcription factor activity, RNA polymerase II-specific"
}